{
  "gene_name": "Transcription factor Sp8",
  "gene_symbol": "SP8",
  "term_label": "RNA polymerase II cis-regulatory region sequence-specific DNA binding",
  "term_id": "GO:0000978",
  "gene": "UniProtKB:Q8IXZ3"
}